{
  "term_id": "GO:0010976",
  "gene_name": "BDNF_NT-3 growth factors receptor",
  "gene_symbol": "NTRK2",
  "term_label": "positive regulation of neuron projection development",
  "gene": "UniProtKB:Q16620"
}